{
  "term_label": "endoplasmic reticulum membrane",
  "gene": "UniProtKB:O76024",
  "gene_symbol": "WFS1",
  "term_id": "GO:0005789",
  "gene_name": "Wolframin"
}